{
  "gene": "UniProtKB:A8MT70",
  "term_label": "Unknown molecular function",
  "term_id": "UNKNOWN:0001",
  "gene_symbol": "ZBBX",
  "gene_name": "Zinc finger B-box domain-containing protein 1"
}